{
  "term_label": "mRNA binding",
  "term_id": "GO:0003729",
  "gene": "UniProtKB:Q9BZI7",
  "gene_name": "Regulator of nonsense transcripts 3B",
  "gene_symbol": "UPF3B"
}